negative regulation of dendritic cell apoptotic process [GO:2000669] (biological process) Sources: GOC:mtg_apoptosis, GOC:obol Definition: Any process that stops, prevents or reduces the frequency, rate or extent of dendritic cell apoptotic process. Relationships: is a type of negative regulation of leukocyte apoptotic process [GO:2000107]; is a type of regulation of dendritic cell apoptotic process [GO:2000668]; negatively regulates dendritic cell apoptotic process [GO:0097048] Also known as: negative regulation of dendritic cell apoptosis